{
  "gene": "UniProtKB:Q96A65",
  "gene_name": "Exocyst complex component 4",
  "term_id": "UNKNOWN:0001",
  "gene_symbol": "EXOC4",
  "term_label": "Unknown molecular function"
}